{
  "gene_symbol": "PAM16",
  "gene": "UniProtKB:Q9Y3D7",
  "gene_name": "Mitochondrial import inner membrane translocase subunit TIM16",
  "term_id": "GO:0005744",
  "term_label": "TIM23 mitochondrial import inner membrane translocase complex"
}